cell junction maintenance [GO:0034331] (biological process) Definition: The organization process that preserves a cell junction in a stable functional or structural state. A cell junction is a specialized region of connection between two cells or between a cell and the extracellular matrix. Sources: GOC:dph, GOC:jl, GOC:mah Relationships: is_a cell junction organization [GO:0034330]; is a type of cellular component maintenance [GO:0043954] Subtypes: cell-cell junction maintenance [GO:0045217], GO:0099558